{
  "gene_name": "Intermediate filament family orphan 2",
  "gene_symbol": "IFFO2",
  "term_label": "Unknown molecular function",
  "gene": "UniProtKB:Q5TF58",
  "term_id": "UNKNOWN:0001"
}